{
  "gene_name": "Coiled-coil domain-containing protein 184",
  "term_label": "cytoplasm",
  "gene_symbol": "CCDC184",
  "gene": "UniProtKB:Q52MB2",
  "term_id": "GO:0005737"
}